{
  "term_label": "Unknown molecular function",
  "gene_name": "Kelch repeat and BTB domain-containing protein 4",
  "gene": "UniProtKB:Q9NVX7",
  "term_id": "UNKNOWN:0001",
  "gene_symbol": "KBTBD4"
}